sorting endosome [GO:0097443] (cellular component) Sources: NIF_Subcellular:sao1028571114 Definition: A multivesicular body surrounded by and connected with multiple tubular compartments with associated vesicles. Also known as: MVB-tubule complex Relationships: is a type of endosome [GO:0005768]